{
  "gene": "UniProtKB:A0A075B6Y3",
  "term_label": "Unknown cellular component",
  "gene_name": "T cell receptor alpha joining 3",
  "term_id": "UNKNOWN:0003",
  "gene_symbol": "TRAJ3"
}